axonemal central bridge [GO:1990717] (cellular component) Definition: Part of the 9+2 axoneme, that occurs in most motile cilia, consisting of the two bridges which connect the central pair of single microtubules. References: PMID:21586547, PMID:9295136 Sources: GOC:cilia Relationships: is a type of cellular anatomical structure [GO:0110165]; is part of axonemal central apparatus [GO:1990716]